{
  "term_id": "GO:0031146",
  "gene_symbol": "FBXO2",
  "term_label": "SCF-dependent proteasomal ubiquitin-dependent protein catabolic process",
  "gene_name": "F-box only protein 2",
  "gene": "UniProtKB:Q9UK22"
}